{
  "gene_name": "T cell receptor gamma constant 2",
  "gene": "UniProtKB:P03986",
  "term_label": "Unknown molecular function",
  "term_id": "UNKNOWN:0001",
  "gene_symbol": "TRGC2"
}